{
  "gene_name": "Putative uncharacterized protein FLJ45275, mitochondrial",
  "gene_symbol": "Q6ZSR3",
  "term_label": "Unknown biological process",
  "gene": "UniProtKB:Q6ZSR3",
  "term_id": "UNKNOWN:0002"
}